{
  "gene_name": "Putative uncharacterized protein C1orf220",
  "gene_symbol": "C1orf220",
  "term_label": "Unknown cellular component",
  "term_id": "UNKNOWN:0003",
  "gene": "UniProtKB:Q5T0J3"
}